{
  "gene_name": "Glycoprotein integral membrane protein 1",
  "term_id": "UNKNOWN:0002",
  "term_label": "Unknown biological process",
  "gene_symbol": "GINM1",
  "gene": "UniProtKB:Q9NU53"
}